{
  "term_id": "UNKNOWN:0001",
  "gene": "UniProtKB:Q8NFQ6",
  "gene_symbol": "BPIFC",
  "term_label": "Unknown molecular function",
  "gene_name": "BPI fold-containing family C protein"
}